{
  "term_id": "GO:0019838",
  "gene_name": "Mast_stem cell growth factor receptor Kit",
  "gene": "UniProtKB:P10721",
  "term_label": "growth factor binding",
  "gene_symbol": "KIT"
}